[methyl-Co(III) methanol-specific corrinoid protein]:coenzyme M methyltransferase [GO:1990088] (molecular function) Definition: Catalysis of the reaction: a [methyl-Co(III) methanol-specific corrinoid protein] + coenzyme M = methyl-coenzyme M + a [Co(I) methanol-specific corrinoid protein] + H+. Note: This function is the second step in the pathway of methanogenesis from methanol. Also known as: methylcobamide:CoM methyltransferase activity, methylcobamide:coenzyme M methyltransferase activity, methanol-specific methylcobalamin: coenzyme M methyltransferase activity, methanol-specific methylcobalamin:CoM methyltransferase activity, methanol-specific methylcobalamin:coenzyme M methyltransferase activity References: PMID:10077852 Sources: GOC:hjd, RHEA:45208 Relationships: is a type of methyltransferase activity [GO:0008168]